{
  "gene_name": "Potassium channel subfamily K member 16",
  "gene": "UniProtKB:Q96T55",
  "gene_symbol": "KCNK16",
  "term_label": "potassium ion leak channel activity",
  "term_id": "GO:0022841"
}